{
  "term_label": "JNK cascade",
  "gene_name": "Mitogen-activated protein kinase kinase kinase 12",
  "gene_symbol": "MAP3K12",
  "term_id": "GO:0007254",
  "gene": "UniProtKB:Q12852"
}